pons reticulospinal tract morphogenesis [GO:0021975] (biological process) Sources: GOC:cls, GOC:dgh, GOC:dph, GOC:jid, GO_REF:0000021 Definition: Generation of a long process of a CNS neuron, that carries efferent (outgoing) action potentials from the cell body in the pons towards target cells in the spinal cord. Relationships: is a type of central nervous system projection neuron axonogenesis [GO:0021952]